{
  "gene_symbol": "TRPV4",
  "term_id": "GO:0098703",
  "term_label": "calcium ion import across plasma membrane",
  "gene": "UniProtKB:Q9HBA0",
  "gene_name": "Transient receptor potential cation channel subfamily V member 4"
}